{
  "term_label": "enzyme inhibitor activity",
  "gene_name": "Protein phosphatase 1 regulatory subunit 12B",
  "gene": "UniProtKB:O60237",
  "gene_symbol": "PPP1R12B",
  "term_id": "GO:0004857"
}